negative regulation of establishment of RNA localization to telomere [GO:1904911] (biological process) References: PMID:26586433 Sources: GOC:BHF, GOC:BHF_telomere, GOC:TermGenie, GOC:rph, GO_REF:0000058 Also known as: down regulation of establishment of RNA localisation to telomere, down regulation of establishment of RNA localization to telomere, down-regulation of establishment of RNA localisation to telomere, down-regulation of establishment of RNA localization to telomere, downregulation of establishment of RNA localisation to telomere, downregulation of establishment of RNA localization to telomere, negative regulation of establishment of RNA localisation to telomere, inhibition of establishment of RNA localisation to telomere, inhibition of establishment of RNA localization to telomere Definition: Any process that stops, prevents or reduces the frequency, rate or extent of establishment of RNA localization to telomere. Relationships: is a type of negative regulation of biological process [GO:0048519]; is a type of GO:1904910; negatively regulates GO:0097694